{
  "gene": "UniProtKB:A0A2R8Y4L6",
  "gene_name": "Olfactory receptor",
  "term_label": "olfactory receptor activity",
  "term_id": "GO:0004984",
  "gene_symbol": "OR5D3"
}